{
  "gene_name": "Zinc finger CCHC domain-containing protein 12",
  "gene_symbol": "ZCCHC12",
  "gene": "UniProtKB:Q6PEW1",
  "term_id": "UNKNOWN:0002",
  "term_label": "Unknown biological process"
}